{
  "term_label": "detection of chemical stimulus involved in sensory perception of smell",
  "gene_symbol": "OR10G8",
  "gene_name": "Olfactory receptor 10G8",
  "gene": "UniProtKB:Q8NGN5",
  "term_id": "GO:0050911"
}